{
  "term_id": "GO:0004756",
  "gene": "UniProtKB:P49903",
  "gene_symbol": "SEPHS1",
  "term_label": "selenide, water dikinase activity",
  "gene_name": "Selenide, water dikinase 1"
}